ABC-type D-allose transporter activity [GO:0015615] (molecular function) Definition: Enables the transfer of a solute or solutes from one side of a membrane to the other according to the reaction: ATP + H2O + D-allose(out) = ADP + phosphate + D-allose(in). Relationships: is a type of hexose transmembrane transporter activity [GO:0015149]; is a type of ABC-type monosaccharide transporter activity [GO:0015407]; is part of D-allose transmembrane transport [GO:0015754] Also known as: D-allose porter activity, D-allose-importing ATPase activity References: PMID:9401019 Sources: RHEA:29799